regulation of melanocyte differentiation [GO:0045634] (biological process) Definition: Any process that modulates the frequency, rate or extent of melanocyte differentiation. Sources: GOC:go_curators Also known as: regulation of melanophore differentiation Relationships: is a type of regulation of pigment cell differentiation [GO:0050932]; regulates melanocyte differentiation [GO:0030318] Subtypes: negative regulation of melanocyte differentiation [GO:0045635], positive regulation of melanocyte differentiation [GO:0045636], regulation of early stripe melanocyte differentiation [GO:0050939], regulation of late stripe melanocyte differentiation [GO:0050940]